positive regulation of xylan catabolic process [GO:2001002] (biological process) Definition: Any process that activates or increases the frequency, rate or extent of xylan catabolic process. Relationships: is a type of positive regulation of hemicellulose catabolic process [GO:2000990]; is a type of regulation of xylan catabolic process [GO:2001000]; positively regulates xylan catabolic process [GO:0045493] Subtypes: GO:2000917, positive regulation of arabinoxylan-containing compound catabolic process [GO:2000923] Also known as: positive regulation of xylan breakdown, positive regulation of xylan catabolism, positive regulation of xylan degradation Sources: GOC:mengo_curators